{
  "term_label": "cytoplasm",
  "gene_name": "PRAME family member 4",
  "gene_symbol": "PRAMEF4",
  "gene": "UniProtKB:O60810",
  "term_id": "GO:0005737"
}